{
  "term_id": "GO:0034587",
  "gene_symbol": "PIWIL2",
  "gene_name": "Piwi-like protein 2",
  "term_label": "piRNA processing",
  "gene": "UniProtKB:Q8TC59"
}